{
  "term_label": "extracellular space",
  "term_id": "GO:0005615",
  "gene_name": "von Willebrand factor",
  "gene_symbol": "VWF",
  "gene": "UniProtKB:P04275"
}